proteinoplast [GO:0031986] (cellular component) Definition: A leucoplast in which protein is stored. Relationships: is a type of GO:0009516 Sources: GOC:pz